{
  "gene": "UniProtKB:Q1MSJ5",
  "term_label": "Unknown molecular function",
  "gene_name": "Centrosome and spindle pole-associated protein 1",
  "gene_symbol": "CSPP1",
  "term_id": "UNKNOWN:0001"
}